{
  "gene": "UniProtKB:A6PVL3",
  "term_id": "GO:0043025",
  "term_label": "neuronal cell body",
  "gene_name": "Kinocilin",
  "gene_symbol": "KNCN"
}